{
  "gene_symbol": "PGD",
  "gene": "UniProtKB:P52209",
  "gene_name": "6-phosphogluconate dehydrogenase, decarboxylating",
  "term_id": "GO:0009051",
  "term_label": "pentose-phosphate shunt, oxidative branch"
}